{
  "term_id": "UNKNOWN:0003",
  "gene": "UniProtKB:Q8NGG2",
  "gene_symbol": "OR5T2",
  "term_label": "Unknown cellular component",
  "gene_name": "Olfactory receptor 5T2"
}